{
  "gene_name": "Lysine-specific demethylase PHF2",
  "term_label": "histone demethylase activity",
  "gene": "UniProtKB:O75151",
  "gene_symbol": "PHF2",
  "term_id": "GO:0032452"
}